DNA exonuclease activity [GO:0004529] (molecular function) Definition: Catalysis of the sequential cleavage of mononucleotides from a free 5' or 3' terminus of a DNA molecule. Subtypes: DNA exonuclease activity, producing 5'-phosphomonoesters [GO:0016895] Sources: GOC:mah, ISBN:0198547684 Relationships: is a type of exonuclease activity [GO:0004527]; is a type of DNA nuclease activity [GO:0004536]